terminal loop [GO:0097456] (cellular component) Relationships: is a type of glial cell projection [GO:0097386] Sources: NIF_Subcellular:sao924713546 Definition: Portion of myelin-forming Schwann cell consisting of terminal cytoplasmic extensions adhered to the axon at the beginning and end of the myelin sheath. Also known as: terminal loop of Schwann cell